{
  "term_label": "lysosomal membrane",
  "gene_symbol": "HPS4",
  "term_id": "GO:0005765",
  "gene": "UniProtKB:Q9NQG7",
  "gene_name": "BLOC-3 complex member HPS4"
}